radial spoke base 2 [GO:0120341] (cellular component) Definition: The short portion of the radial spoke 2 (RS2) that is directly anchored to the A microtubule of an axonemal microtubule doublet. References: PMID:22754630, PMID:25694453 Sources: GOC:krc Relationships: is a type of GO:0120339; is part of radial spoke 2 [GO:0120334]